{
  "gene_symbol": "OR5M11",
  "gene": "UniProtKB:Q96RB7",
  "gene_name": "Olfactory receptor 5M11",
  "term_id": "UNKNOWN:0003",
  "term_label": "Unknown cellular component"
}